{
  "gene_name": "Serpin B8",
  "term_label": "cytoplasm",
  "gene": "UniProtKB:P50452",
  "gene_symbol": "SERPINB8",
  "term_id": "GO:0005737"
}